{
  "gene_name": "Translocon-associated protein subunit gamma",
  "gene_symbol": "SSR3",
  "term_label": "Unknown molecular function",
  "term_id": "UNKNOWN:0001",
  "gene": "UniProtKB:Q9UNL2"
}